{
  "gene": "UniProtKB:Q8TBF5",
  "term_id": "UNKNOWN:0001",
  "term_label": "Unknown molecular function",
  "gene_name": "Phosphatidylinositol-glycan biosynthesis class X protein",
  "gene_symbol": "PIGX"
}